erythrocyte enucleation [GO:0043131] (biological process) Relationships: is a type of enucleation [GO:0090601]; is part of enucleate erythrocyte maturation [GO:0043354] Regulation: regulated by regulation of erythrocyte enucleation [GO:0061930]; positively regulated by positive regulation of erythrocyte enucleation [GO:0061931]; negatively regulated by negative regulation of erythrocyte enucleation [GO:0061932] Definition: The process in which nucleated precursor cells lose their nucleus during erythrocyte maturation. Sources: GOC:hjd